{
  "gene": "UniProtKB:P01375",
  "gene_name": "Tumor necrosis factor",
  "gene_symbol": "TNF",
  "term_id": "GO:0006955",
  "term_label": "immune response"
}